{
  "term_id": "GO:0005739",
  "gene_name": "Hydroxyacyl-thioester dehydratase type 2, mitochondrial",
  "gene": "UniProtKB:P86397",
  "gene_symbol": "HTD2",
  "term_label": "mitochondrion"
}